{
  "gene_symbol": "PRKN",
  "gene_name": "E3 ubiquitin-protein ligase parkin",
  "gene": "UniProtKB:O60260",
  "term_id": "GO:0061630",
  "term_label": "ubiquitin protein ligase activity"
}